{
  "gene": "UniProtKB:Q8TAM6",
  "gene_name": "Ermin",
  "gene_symbol": "ERMN",
  "term_label": "cell cortex",
  "term_id": "GO:0005938"
}